{
  "gene_name": "Beta-1,3-galactosyltransferase 5",
  "term_label": "Golgi membrane",
  "term_id": "GO:0000139",
  "gene_symbol": "B3GALT5",
  "gene": "UniProtKB:Q9Y2C3"
}